GDP-mannose 3,5-epimerase activity [GO:0047918] (molecular function) Also known as: GDP-D-mannose:GDP-L-galactose epimerase activity, GDPmannose 3,5-epimerase activity, guanosine 5'-diphosphate D-mannose:guanosine 5'-diphosphate L-galactose epimerase activity Definition: Catalysis of the reaction: GDP-mannose = GDP-L-galactose. References: PMID:16366586, PMID:8910301 Relationships: is a type of racemase and epimerase activity, acting on carbohydrates and derivatives [GO:0016857]